lipoteichoic acid D-alanylation [GO:0036358] (biological process) Relationships: is a type of teichoic acid D-alanylation [GO:0070400] Definition: The formation of a D-alanyl ester of lipoteichoic acid by transfer of D-Ala onto a membrane-associated lipoteichoic acid (LTA). Also known as: D-alanyl LTA formation, D-alanyl lipoteichoic acid formation, LTA D-alanylation References: PMID:22750871, PMID:8682792 Sources: GOC:crds